{
  "gene_name": "Inositol 1,4,5-trisphosphate receptor type 3",
  "gene_symbol": "ITPR3",
  "gene": "UniProtKB:Q14573",
  "term_id": "GO:0005789",
  "term_label": "endoplasmic reticulum membrane"
}